NLRP3 inflammasome complex [GO:0072559] (cellular component) Definition: An inflammasome complex that consists of three components, NLRP3 (NALP3), PYCARD and caspase-1. It is activated upon exposure to whole pathogens, as well as a number of structurally diverse pathogen- and danger-associated molecular patterns (PAMPs and DAMPs) and environmental irritants. Whole pathogens demonstrated to activate the NLRP3 inflammasome complex include the fungi Candida albicans and Saccharomyces cerevisiae, bacteria that produce pore-forming toxins, including Listeria monocytogenes and Staphylococcus aureus, and viruses such as Sendai virus, adenovirus, and influenza virus. References: PMID:20303873 Sources: GOC:BHF, GOC:add, GOC:vp Also known as: NALP3 inflammasome complex Relationships: is a type of canonical inflammasome complex [GO:0061702]